{
  "gene": "UniProtKB:P15336",
  "gene_name": "Cyclic AMP-dependent transcription factor ATF-2",
  "gene_symbol": "ATF2",
  "term_id": "GO:0006357",
  "term_label": "regulation of transcription by RNA polymerase II"
}